vestibulocochlear nerve morphogenesis [GO:0021648] (biological process) Relationships: is a type of cranial nerve morphogenesis [GO:0021602]; is part of vestibulocochlear nerve development [GO:0021562] Also known as: CN VIII morphogenesis Definition: The process in which the anatomical structure of the vestibulocochlear nerve is generated and organized. This sensory nerve innervates the membranous labyrinth of the inner ear. The vestibular branch innervates the vestibular apparatus that senses head position changes relative to gravity. The auditory branch innervates the cochlear duct, which is connected to the three bony ossicles which transduce sound waves into fluid movement in the cochlea. Sources: GOC:cls, GOC:dgh, GOC:dph, GOC:jid, GO_REF:0000021